{
  "term_id": "UNKNOWN:0003",
  "term_label": "Unknown cellular component",
  "gene": "UniProtKB:Q499Z3",
  "gene_symbol": "SLFNL1",
  "gene_name": "Schlafen-like protein 1"
}